{
  "term_id": "GO:0004065",
  "term_label": "arylsulfatase activity",
  "gene_symbol": "ARSF",
  "gene": "UniProtKB:P54793",
  "gene_name": "Arylsulfatase F"
}